response to axon injury [GO:0048678] (biological process) Relationships: is a type of response to wounding [GO:0009611] Definition: Any process that results in a change in state or activity of a cell or an organism (in terms of movement, secretion, enzyme production, gene expression, etc.) as a result of an axon injury stimulus. Sources: GOC:dgh, GOC:dph, GOC:jid, GOC:lm Subtypes: axon regeneration [GO:0031103]